{
  "gene_name": "Transcriptional enhancer factor TEF-1",
  "gene": "UniProtKB:P28347",
  "term_label": "RNA polymerase II cis-regulatory region sequence-specific DNA binding",
  "gene_symbol": "TEAD1",
  "term_id": "GO:0000978"
}